{
  "gene_symbol": "IKBKE",
  "term_id": "GO:0002218",
  "term_label": "activation of innate immune response",
  "gene_name": "Inhibitor of nuclear factor kappa-B kinase subunit epsilon",
  "gene": "UniProtKB:Q14164"
}